{
  "gene_symbol": "RBKS",
  "term_label": "Unknown biological process",
  "gene": "UniProtKB:Q9H477",
  "term_id": "UNKNOWN:0002",
  "gene_name": "Ribokinase"
}